regulation of release of cytochrome c from mitochondria [GO:0090199] (biological process) Subtypes: positive regulation of release of cytochrome c from mitochondria [GO:0090200], GO:0090201 Definition: Any process that modulates the rate, frequency or extent of release of cytochrome c from mitochondria, the process in which cytochrome c is enabled to move from the mitochondrial intermembrane space into the cytosol, which is an early step in apoptosis and leads to caspase activation. Relationships: is a type of regulation of mitochondrion organization [GO:0010821]; regulates release of cytochrome c from mitochondria [GO:0001836] Sources: GOC:dph, GOC:mtg_apoptosis, GOC:tb Note: The release of cytochrome c from mitochondria is a central event in the signaling phase of the apoptotic process, and it is often used by researchers to monitor this type of cell death. Any event that induces apoptosis will at some point induce the release of cytochrome c from mitochondria. Therefore, this term should only be used to annotate gene products that directly regulate this process.